bis(5'-adenosyl)-triphosphatase activity [GO:0047710] (molecular function) Also known as: 1-P,3-P-bis(5'-adenosyl)-triphosphate adenylohydrolase activity, AP(3)A hydrolase activity, AP(3)Aase activity, AP3A hydrolase activity, AP3Aase activity, P1,P3-bis(5'-adenosyl)-triphosphate adenylohydrolase activity, diadenosine 5',5'''-P(1),P(3)-triphosphate hydrolase activity, diadenosine 5',5'''-P1,P3-triphosphate hydrolase activity, diadenosine 5,5-P1,P3-triphosphatase activity, dinucleosidetriphosphatase activity Sources: EC:3.6.1.29, RHEA:13893 Relationships: is a type of pyrophosphatase activity [GO:0016462] Definition: Catalysis of the reaction: P(1),P(3)-bis(5'-adenosyl) triphosphate + H2O = ADP + AMP + 2 H+.